{
  "term_label": "Unknown biological process",
  "term_id": "UNKNOWN:0002",
  "gene": "UniProtKB:Q9H008",
  "gene_symbol": "LHPP",
  "gene_name": "Phospholysine phosphohistidine inorganic pyrophosphate phosphatase"
}